{
  "term_label": "neuron projection",
  "gene_symbol": "GPR149",
  "gene": "UniProtKB:Q86SP6",
  "gene_name": "Probable G-protein coupled receptor 149",
  "term_id": "GO:0043005"
}